neuromuscular synaptic transmission [GO:0007274] (biological process) Subtypes: synaptic transmission involved in micturition [GO:0060084] Regulation: regulated by regulation of neuromuscular synaptic transmission [GO:1900073]; negatively regulated by negative regulation of neuromuscular synaptic transmission [GO:1900074]; positively regulated by positive regulation of neuromuscular synaptic transmission [GO:1900075] Definition: The process of synaptic transmission from a neuron to a muscle, across a synapse. Relationships: is_a chemical synaptic transmission [GO:0007268] Sources: GOC:dos, GOC:jl, MeSH:D009435